clathrin-coated vesicle cargo loading [GO:0035652] (biological process) Definition: Formation of a macromolecular complex between the cytoplasmic coat proteins on clathrin-coated vesicles and proteins and/or lipoproteins that are going to be transported by a vesicle. Also known as: cargo loading into clathrin-coated vesicle Relationships: is a type of vesicle cargo loading [GO:0035459] References: PMID:16162817 Sources: GOC:lb Subtypes: clathrin-coated vesicle cargo loading, AP-1-mediated [GO:0035653], clathrin-coated vesicle cargo loading, AP-3-mediated [GO:0035654], cargo loading involved in clathrin-dependent endocytosis [GO:0099043]